B cell anergy [GO:0002515] (biological process) Relationships: is a type of lymphocyte anergy [GO:0002249]; is_a GO:0002514 Sources: GOC:jal, ISBN:0781735149 Subtypes: GO:0002341, GO:0002453 Also known as: B lymphocyte anergy, B-cell anergy, B-lymphocyte anergy Regulation: regulated by regulation of B cell anergy [GO:0002670]; negatively regulated by negative regulation of B cell anergy [GO:0002671]; positively regulated by positive regulation of B cell anergy [GO:0002672] Definition: Any process contributing to anergy in B cells, a state of functional inactivation which is part of B cell tolerance induction.